{
  "term_id": "GO:0048188",
  "gene": "UniProtKB:O15047",
  "term_label": "Set1C/COMPASS complex",
  "gene_name": "Histone-lysine N-methyltransferase SETD1A",
  "gene_symbol": "SETD1A"
}